purine ribonucleoside bisphosphate metabolic process [GO:0034035] (biological process) Definition: The chemical reactions and pathways involving a purine ribonucleoside bisphosphate, a compound consisting of a purine base linked to a ribose sugar esterified with one phosphate group attached to each of two different hydroxyl groups on the sugar. Sources: GOC:mah, GOC:pde Also known as: purine ribonucleoside bisphosphate metabolism Relationships: is a type of ribonucleoside bisphosphate metabolic process [GO:0033875]; is a type of purine nucleoside bisphosphate metabolic process [GO:0034032] Subtypes: guanosine tetraphosphate metabolic process [GO:0015969], GO:0015972, purine ribonucleoside bisphosphate biosynthetic process [GO:0034036], purine ribonucleoside bisphosphate catabolic process [GO:0034037], 3'-phosphoadenosine 5'-phosphosulfate metabolic process [GO:0050427]